{
  "term_id": "GO:0035722",
  "gene_name": "Interleukin-12 subunit beta",
  "term_label": "interleukin-12-mediated signaling pathway",
  "gene": "UniProtKB:P29460",
  "gene_symbol": "IL12B"
}